{
  "gene_name": "Fanconi anemia group J protein",
  "gene": "UniProtKB:Q9BX63",
  "gene_symbol": "BRIP1",
  "term_label": "nucleus",
  "term_id": "GO:0005634"
}